L-2-hydroxycarboxylate dehydrogenase (NAD+) activity [GO:0102443] (MF) Definition: Catalysis of the reaction: a (2S)-2-hydroxycarboxylate + NAD+ = a 2-oxocarboxylate + NADH + H+. Relationships: is a type of oxidoreductase activity, acting on the CH-OH group of donors, NAD or NADP as acceptor [GO:0016616] Sources: RHEA:34555 Subtypes: L-lactate dehydrogenase (NAD+) activity [GO:0004459]